{
  "gene_symbol": "ATP11C",
  "gene_name": "Phospholipid-transporting ATPase IG",
  "term_id": "GO:0045332",
  "term_label": "phospholipid translocation",
  "gene": "UniProtKB:Q8NB49"
}